{
  "term_label": "peroxisomal membrane",
  "gene_name": "Peroxisomal membrane protein PEX13",
  "gene_symbol": "PEX13",
  "term_id": "GO:0005778",
  "gene": "UniProtKB:Q92968"
}